{
  "gene_name": "Integrin alpha-M",
  "term_id": "GO:0009986",
  "gene": "UniProtKB:P11215",
  "term_label": "cell surface",
  "gene_symbol": "ITGAM"
}